{
  "gene": "UniProtKB:Q2VY69",
  "term_id": "GO:0000981",
  "term_label": "DNA-binding transcription factor activity, RNA polymerase II-specific",
  "gene_symbol": "ZNF284",
  "gene_name": "Zinc finger protein 284"
}